arg-arg specific dibasic protein processing [GO:0090474] (biological process) Sources: GOC:al Relationships: is_a GO:0090472 Definition: Any protein processing achieved by the cleavage of a peptide bond after two consecutive arginine amino acid residues within a protein.